chemical synaptic transmission [GO:0007268] (biological process) Also known as: signal transmission across a synapse, synaptic transmission, neurotransmission Subtypes: GO:0001963, neuron-neuron synaptic transmission [GO:0007270], GO:0007271, neuromuscular synaptic transmission [GO:0007274], synaptic transmission, glutamatergic [GO:0035249], synaptic transmission, GABAergic [GO:0051932], GO:0060012, GO:0090127, GO:0098814, excitatory chemical synaptic transmission [GO:0098976], inhibitory chemical synaptic transmission [GO:0098977], synaptic transmission, serotonergic [GO:0099153], synaptic transmission, noradrenergic [GO:0099155] Sources: GOC:jl, MeSH:D009435 Definition: The vesicular release of classical neurotransmitter molecules from a presynapse, across a chemical synapse, the subsequent activation of neurotransmitter receptors at the postsynapse of a target cell (neuron, muscle, or secretory cell) and the effects of this activation on the postsynaptic membrane potential and ionic composition of the postsynaptic cytosol. This process encompasses both spontaneous and evoked release of neurotransmitter and all parts of synaptic vesicle exocytosis. Evoked transmission starts with the arrival of an action potential at the presynapse. Relationships: is_a anterograde trans-synaptic signaling [GO:0098916] Regulation: regulated by modulation of chemical synaptic transmission [GO:0050804]; negatively regulated by GO:0050805; positively regulated by positive regulation of synaptic transmission [GO:0050806]; regulated by GO:0099546; regulated by modification of synaptic structure, modulating synaptic transmission [GO:0099564]; regulated by GO:0140237